{
  "gene_name": "Serine_threonine-protein kinase MRCK beta",
  "gene": "UniProtKB:Q9Y5S2",
  "term_id": "GO:0042641",
  "term_label": "actomyosin",
  "gene_symbol": "CDC42BPB"
}